{
  "gene_symbol": "TLE3",
  "term_label": "nucleus",
  "gene": "UniProtKB:Q04726",
  "term_id": "GO:0005634",
  "gene_name": "Transducin-like enhancer protein 3"
}